{
  "gene_name": "Cdc42 effector protein 1",
  "term_label": "small GTPase binding",
  "term_id": "GO:0031267",
  "gene_symbol": "CDC42EP1",
  "gene": "UniProtKB:Q00587"
}